{
  "term_label": "endoplasmic reticulum",
  "gene_name": "Long-chain-fatty-acid--CoA ligase 6",
  "term_id": "GO:0005783",
  "gene": "UniProtKB:Q9UKU0",
  "gene_symbol": "ACSL6"
}